{
  "term_label": "centrosome",
  "gene": "UniProtKB:Q96GD4",
  "gene_symbol": "AURKB",
  "gene_name": "Aurora kinase B",
  "term_id": "GO:0005813"
}